mitochondrial citrate transmembrane transport [GO:0006843] (biological process) Relationships: is a type of citrate transport [GO:0015746]; is a type of mitochondrial tricarboxylic acid transmembrane transport [GO:1990546] References: PMID:20371607 Sources: GOC:ai Definition: The directed movement of citrate, 2-hydroxy-1,2,3-propanetricarboxylate, into or out of a mitochondrial matrix. Also known as: mitochondrial citrate transport